{
  "term_label": "axon guidance",
  "gene_symbol": "EFNA2",
  "gene_name": "Ephrin-A2",
  "term_id": "GO:0007411",
  "gene": "UniProtKB:O43921"
}